{
  "term_id": "GO:0006633",
  "gene_name": "Acyl-coenzyme A synthetase ACSM2B, mitochondrial",
  "term_label": "fatty acid biosynthetic process",
  "gene_symbol": "ACSM2B",
  "gene": "UniProtKB:Q68CK6"
}